{
  "term_label": "nucleus",
  "gene_name": "NSFL1 cofactor p47",
  "gene_symbol": "NSFL1C",
  "term_id": "GO:0005634",
  "gene": "UniProtKB:Q9UNZ2"
}